{
  "gene_name": "Ras-related protein Rab-6C",
  "gene": "UniProtKB:Q9H0N0",
  "term_id": "GO:1903292",
  "gene_symbol": "RAB6C",
  "term_label": "protein localization to Golgi membrane"
}